light-harvesting complex [GO:0030076] (cellular component) Sources: GOC:lr Also known as: antenna complex Subtypes: thylakoid light-harvesting complex [GO:0009503], plasma membrane light-harvesting complex [GO:0030077], GO:0030089 Definition: A protein-pigment complex that may be closely or peripherally associated to photosynthetic reaction centers that participate in harvesting and transferring radiant energy to the reaction center. Relationships: is a type of protein-containing complex [GO:0032991]; is part of intracellular anatomical structure [GO:0005622]